{
  "gene_name": "Beta-1,3-galactosyl-O-glycosyl-glycoprotein beta-1,6-N-acetylglucosaminyltransferase 3",
  "term_label": "acetylglucosaminyltransferase activity",
  "term_id": "GO:0008375",
  "gene_symbol": "GCNT3",
  "gene": "UniProtKB:O95395"
}